{
  "term_label": "Unknown cellular component",
  "gene_name": "Tyrosine-protein phosphatase non-receptor type 14",
  "gene": "UniProtKB:Q15678",
  "term_id": "UNKNOWN:0003",
  "gene_symbol": "PTPN14"
}